protein localization to cleavage furrow [GO:1905345] (biological process) Definition: A process in which a protein is transported to, or maintained in, a location within a cleavage furrow. Relationships: is a type of GO:0072657; is a type of protein localization to cell division site [GO:0072741]; is a type of protein localization to cell periphery [GO:1990778] References: PMID:27082518 Sources: GOC:TermGenie, GO_REF:0000087 Also known as: protein localisation in cleavage furrow, protein localisation to cleavage furrow, protein localization in cleavage furrow Subtypes: protein localization to cleavage furrow rim [GO:1905346]